cell-substrate adhesion [GO:0031589] (biological process) Definition: The attachment of a cell to the underlying substrate via adhesion molecules. Sources: GOC:mah, GOC:pf Subtypes: substrate-dependent cell migration, cell attachment to substrate [GO:0006931], cell-matrix adhesion [GO:0007160], cell-matrix adhesion involved in tangential migration using cell-cell interactions [GO:0021833], interneuron-substratum interaction involved in interneuron migration from the subpallium to the cortex [GO:0021839], substrate adhesion-dependent cell spreading [GO:0034446], cell-abiotic substrate adhesion [GO:0036164], cell adhesion involved in biofilm formation [GO:0043708] Regulation: regulated by GO:0010810; positively regulated by positive regulation of cell-substrate adhesion [GO:0010811]; negatively regulated by negative regulation of cell-substrate adhesion [GO:0010812] Relationships: is a type of cell adhesion [GO:0007155]